2-dehydropantolactone reductase activity [GO:0036441] (molecular function) Sources: RHEA:18981 Definition: Catalysis of the reaction: (R)-pantolactone + NADP+ = 2-dehydropantolactone + NADPH + H+. Subtypes: 2-dehydropantolactone reductase (B-specific) activity [GO:0019141], 2-dehydropantolactone reductase (A-specific) activity [GO:0047011] Relationships: is a type of oxidoreductase activity, acting on the CH-OH group of donors, NAD or NADP as acceptor [GO:0016616]